solute:inorganic anion antiporter activity [GO:0005452] (molecular function) Definition: Enables the transfer of a solute or solutes from one side of a membrane to the other according to the reaction: inorganic anion(out) + solute(in) = inorganic anion (in) + solute(out). Sources: GOC:mah Also known as: inorganic anion exchanger activity Relationships: is a type of antiporter activity [GO:0015297] Subtypes: organophosphate:phosphate antiporter activity [GO:0015315], dicarboxylate:phosphate antiporter activity [GO:0015364], sulfate:bicarbonate antiporter activity [GO:0015383], chloride:proton antiporter activity [GO:0062158], chloride:bicarbonate antiporter activity [GO:0140900], sulfate:chloride antiporter activity [GO:0160044], oxalate:chloride antiporter activity [GO:0160046]